{
  "gene": "UniProtKB:Q8N6T3",
  "term_id": "GO:0000139",
  "term_label": "Golgi membrane",
  "gene_symbol": "ARFGAP1",
  "gene_name": "ADP-ribosylation factor GTPase-activating protein 1"
}